{
  "gene_name": "ARF GTPase-activating protein GIT1",
  "term_id": "GO:0031267",
  "gene": "UniProtKB:Q9Y2X7",
  "term_label": "small GTPase binding",
  "gene_symbol": "GIT1"
}